{
  "term_id": "GO:0005861",
  "term_label": "troponin complex",
  "gene": "UniProtKB:P13805",
  "gene_symbol": "TNNT1",
  "gene_name": "Troponin T, slow skeletal muscle"
}